{
  "term_id": "GO:0004252",
  "gene_name": "Rhomboid domain-containing protein 3",
  "gene": "UniProtKB:Q9Y3P4",
  "gene_symbol": "RHBDD3",
  "term_label": "serine-type endopeptidase activity"
}